{
  "gene_symbol": "CXCL9",
  "gene_name": "C-X-C motif chemokine 9",
  "term_id": "GO:0005615",
  "gene": "UniProtKB:Q07325",
  "term_label": "extracellular space"
}